{
  "gene_symbol": "PEAR1",
  "term_label": "membrane",
  "gene": "UniProtKB:Q5VY43",
  "term_id": "GO:0016020",
  "gene_name": "Platelet endothelial aggregation receptor 1"
}